{
  "gene": "UniProtKB:P26038",
  "gene_symbol": "MSN",
  "term_id": "GO:2000643",
  "gene_name": "Moesin",
  "term_label": "positive regulation of early endosome to late endosome transport"
}